nitrogenase activity [GO:0016163] (molecular function) References: PMID:15382920 Sources: RHEA:21448 Relationships: is a type of oxidoreductase activity, acting on iron-sulfur proteins as donors, dinitrogen as acceptor [GO:0016732]; is part of nitrogen fixation [GO:0009399] Also known as: iron-iron nitrogenase activity, molybdenum-iron nitrogenase activity, vanadium-iron nitrogenase activity, reduced ferredoxin:dinitrogen oxidoreductase (ATP-hydrolysing) activity Definition: Catalysis of the reaction: 16 ATP + 16 H2O + N2 + 8 reduced [2Fe-2S]-[ferredoxin] = 16 ADP + 6 H+ + H2 + 2 NH4+ + 8 oxidized [2Fe-2S]-[ferredoxin] + 16 phosphate.